{
  "gene": "UniProtKB:P59826",
  "gene_symbol": "BPIFB3",
  "gene_name": "BPI fold-containing family B member 3",
  "term_id": "UNKNOWN:0001",
  "term_label": "Unknown molecular function"
}